{
  "term_id": "GO:0004984",
  "term_label": "olfactory receptor activity",
  "gene": "UniProtKB:Q8NG84",
  "gene_name": "Olfactory receptor 2AK2",
  "gene_symbol": "OR2AK2"
}